negative regulation of intermediate filament polymerization [GO:0030840] (biological process) Note: Note that this term was split from 'negative regulation of intermediate filament polymerization and/or depolymerization ; GO:0045825' (sibling term 'negative regulation of intermediate filament depolymerization ; GO:0030843'). Definition: Any process that stops, prevents, or reduces the frequency, rate or extent of intermediate filament polymerization. Also known as: negative regulation of intermediate filament polymerization and/or depolymerization, down regulation of intermediate filament polymerization, down-regulation of intermediate filament polymerization, downregulation of intermediate filament polymerization, inhibition of intermediate filament polymerization Sources: GOC:mah Relationships: is a type of regulation of intermediate filament polymerization [GO:0030839]; is a type of negative regulation of protein polymerization [GO:0032272]; is a type of negative regulation of cytoskeleton organization [GO:0051494]; negatively regulates GO:0045107